{
  "term_label": "COP9 signalosome",
  "gene_name": "COP9 signalosome complex subunit 7b",
  "gene": "UniProtKB:Q9H9Q2",
  "gene_symbol": "COPS7B",
  "term_id": "GO:0008180"
}